{
  "term_id": "UNKNOWN:0003",
  "gene_symbol": "PPP1R2",
  "gene_name": "Protein phosphatase inhibitor 2",
  "gene": "UniProtKB:P41236",
  "term_label": "Unknown cellular component"
}